{
  "gene_symbol": "SLC28A1",
  "gene_name": "Sodium_nucleoside cotransporter 1",
  "term_label": "uridine transmembrane transport",
  "gene": "UniProtKB:O00337",
  "term_id": "GO:0015862"
}